formyltetrahydrofolate dehydrogenase activity [GO:0016155] (molecular function) Definition: Catalysis of the reaction: 10-formyltetrahydrofolate + H2O + NADP+ = (6S)-5,6,7,8-tetrahydrofolate + CO2 + H+ + NADPH. Relationships: is a type of oxidoreductase activity, acting on the CH-NH group of donors, NAD or NADP as acceptor [GO:0016646] Also known as: 10-formyl tetrahydrofolate:NADP oxidoreductase activity, 10-formyl-H2PtGlu:NADP oxidoreductase activity, 10-formyl-H4folate dehydrogenase activity, 10-formyltetrahydrofolate dehydrogenase activity, 10-formyltetrahydrofolate:NADP+ oxidoreductase activity, N10-formyltetrahydrofolate dehydrogenase activity Sources: EC:1.5.1.6, RHEA:10180